{
  "gene": "UniProtKB:A0A589",
  "gene_symbol": "TRBV4-3",
  "term_label": "plasma membrane",
  "term_id": "GO:0005886",
  "gene_name": "T cell receptor beta variable 4-3"
}